{
  "gene_name": "Immunoglobulin superfamily member 2",
  "term_label": "membrane",
  "term_id": "GO:0016020",
  "gene_symbol": "CD101",
  "gene": "UniProtKB:Q93033"
}